regulation of astrocyte differentiation [GO:0048710] (biological process) References: PMID:15139015 Sources: GOC:vp Relationships: is a type of GO:0045685; regulates GO:0048708 Definition: Any process that modulates the frequency, rate or extent of astrocyte differentiation. Subtypes: positive regulation of astrocyte differentiation [GO:0048711], negative regulation of astrocyte differentiation [GO:0048712], regulation of astrocyte activation [GO:0061888]